glycoprotein network [GO:0048222] (cellular component) References: PMID:18508691, PMID:7048321 Sources: GOC:mah Relationships: is a type of cellular anatomical structure [GO:0110165]; is part of primary cell wall [GO:0009530] Definition: An extracellular matrix part that consists of cross-linked glycoproteins. Also known as: extensin